{
  "term_label": "cytoplasm",
  "gene_symbol": "QPRT",
  "gene_name": "Nicotinate-nucleotide pyrophosphorylase [carboxylating]",
  "gene": "UniProtKB:Q15274",
  "term_id": "GO:0005737"
}